{
  "gene": "UniProtKB:Q8IWS0",
  "term_id": "GO:0042826",
  "gene_symbol": "PHF6",
  "term_label": "histone deacetylase binding",
  "gene_name": "PHD finger protein 6"
}